modulation by host of viral catalytic activity [GO:0044867] (BP) Subtypes: GO:0044866 Definition: The process in which a host organism effects a change in the enzyme activity of a virus with which it is infected. Sources: GOC:jl Relationships: is_a modulation by host of viral molecular function [GO:0044868]; regulates catalytic activity [GO:0003824]